establishment of pigment granule localization [GO:0051905] (biological process) Sources: GOC:ai Also known as: establishment of pigment granule localisation Subtypes: GO:0032401, pigment granule dispersal [GO:0051876], pigment granule aggregation in cell center [GO:0051877], pigment granule transport [GO:0051904] Definition: The directed movement of a pigment granule to a specific location. Relationships: is a type of establishment of vesicle localization [GO:0051650]; is part of pigment granule localization [GO:0051875]